{
  "gene_symbol": "VCP",
  "term_id": "GO:0097352",
  "gene": "UniProtKB:P55072",
  "gene_name": "Transitional endoplasmic reticulum ATPase",
  "term_label": "autophagosome maturation"
}